{
  "term_id": "GO:0033130",
  "gene": "UniProtKB:P0DP57",
  "term_label": "acetylcholine receptor binding",
  "gene_symbol": "SLURP2",
  "gene_name": "Secreted Ly-6_uPAR domain-containing protein 2"
}